{
  "gene_name": "DnaJ homolog subfamily B member 7",
  "term_label": "nucleus",
  "gene": "UniProtKB:Q7Z6W7",
  "term_id": "GO:0005634",
  "gene_symbol": "DNAJB7"
}